{
  "term_label": "bile acid and bile salt transport",
  "gene_symbol": "SLCO1A2",
  "term_id": "GO:0015721",
  "gene": "UniProtKB:P46721",
  "gene_name": "Solute carrier organic anion transporter family member 1A2"
}